{
  "gene": "UniProtKB:Q8IWB9",
  "gene_name": "Testis-expressed protein 2",
  "term_label": "Unknown biological process",
  "gene_symbol": "TEX2",
  "term_id": "UNKNOWN:0002"
}